{
  "term_id": "GO:0071617",
  "gene": "UniProtKB:Q96N66",
  "term_label": "lysophospholipid acyltransferase activity",
  "gene_symbol": "MBOAT7",
  "gene_name": "Lysophospholipid acyltransferase 7"
}